{
  "gene_symbol": "NPFFR2",
  "gene_name": "Neuropeptide FF receptor 2",
  "term_label": "cellular response to hormone stimulus",
  "gene": "UniProtKB:Q9Y5X5",
  "term_id": "GO:0032870"
}